{
  "gene_symbol": "AURKA",
  "gene": "UniProtKB:O14965",
  "gene_name": "Aurora kinase A",
  "term_id": "GO:0000922",
  "term_label": "spindle pole"
}